cellular response to rhamnose stimulus [GO:0071334] (biological process) Definition: Any process that results in a change in state or activity of a cell (in terms of movement, secretion, enzyme production, gene expression, etc.) as a result of a rhamnose stimulus. Sources: GOC:mah Also known as: cellular response to L-rhamnose stimulus Relationships: is a type of response to rhamnose [GO:0032149]; is a type of cellular response to hexose stimulus [GO:0071331]